{
  "term_id": "GO:0045944",
  "gene_name": "Mothers against decapentaplegic homolog 3",
  "term_label": "positive regulation of transcription by RNA polymerase II",
  "gene": "UniProtKB:P84022",
  "gene_symbol": "SMAD3"
}